positive regulation of calcium ion transport into cytosol involved in cellular response to calcium ion [GO:1901198] (biological process) Relationships: is a type of positive regulation of calcium ion transport into cytosol [GO:0010524]; is part of GO:0071277 Also known as: positive regulation of calcium ion transport into cytosol involved in cellular response to Ca2+ ion Sources: GOC:TermGenie Definition: Any positive regulation of calcium ion transport into cytosol that is involved in cellular response to calcium ion.